{
  "term_id": "UNKNOWN:0001",
  "gene_symbol": "A0A2R8Y4M2",
  "gene": "UniProtKB:A0A2R8Y4M2",
  "term_label": "Unknown molecular function",
  "gene_name": "Uncharacterized protein"
}